{
  "gene_name": "Zinc finger protein 781",
  "gene_symbol": "ZNF781",
  "term_id": "UNKNOWN:0001",
  "term_label": "Unknown molecular function",
  "gene": "UniProtKB:Q8N8C0"
}